asexual spore wall assembly [GO:0042243] (biological process) Relationships: is a type of developmental process involved in reproduction [GO:0003006]; is a type of spore wall assembly [GO:0042244]; is part of asexual sporulation [GO:0030436] Also known as: asexual spore wall formation Definition: The aggregation, arrangement and bonding together of a set of components to form an asexual spore wall, the specialized envelope lying outside the cell membrane of a spore derived from an asexual process. Examples of this process are found in Bacterial and Fungal species. Sources: GOC:mah